{
  "term_id": "GO:0050767",
  "term_label": "regulation of neurogenesis",
  "gene_symbol": "HES6",
  "gene_name": "Transcription cofactor HES-6",
  "gene": "UniProtKB:Q96HZ4"
}